regulation of neural crest cell fate specification [GO:1905295] (biological process) Relationships: is a type of regulation of cell fate specification [GO:0042659]; is a type of regulation of neural crest formation [GO:0090299]; is a type of GO:1905292; regulates neural crest cell fate specification [GO:0014036] Definition: Any process that modulates the frequency, rate or extent of neural crest cell fate specification. References: PMID:15073157 Sources: GOC:BHF, GOC:TermGenie, GOC:rl, GO_REF:0000058 Subtypes: negative regulation of neural crest cell fate specification [GO:1905296], positive regulation of neural crest cell fate specification [GO:1905297]